{
  "gene": "UniProtKB:Q12946",
  "term_label": "DNA-binding transcription factor activity, RNA polymerase II-specific",
  "gene_symbol": "FOXF1",
  "gene_name": "Forkhead box protein F1",
  "term_id": "GO:0000981"
}